{
  "term_label": "midbody",
  "gene": "UniProtKB:Q68DK2",
  "gene_symbol": "ZFYVE26",
  "term_id": "GO:0030496",
  "gene_name": "Zinc finger FYVE domain-containing protein 26"
}